{
  "gene": "UniProtKB:Q14596",
  "term_id": "GO:0000407",
  "term_label": "phagophore assembly site",
  "gene_name": "Next to BRCA1 gene 1 protein",
  "gene_symbol": "NBR1"
}